{
  "term_label": "transmembrane transporter activity",
  "gene_symbol": "SLC25A27",
  "term_id": "GO:0022857",
  "gene": "UniProtKB:O95847",
  "gene_name": "Mitochondrial uncoupling protein 4"
}